{
  "term_id": "GO:0005576",
  "term_label": "extracellular region",
  "gene_name": "Acidic mammalian chitinase",
  "gene": "UniProtKB:Q9BZP6",
  "gene_symbol": "CHIA"
}